{
  "term_id": "GO:0031424",
  "gene_symbol": "KRT86",
  "gene": "UniProtKB:O43790",
  "term_label": "keratinization",
  "gene_name": "Keratin, type II cuticular Hb6"
}